microprocessor complex [GO:0070877] (cellular component) Definition: A protein complex that binds to heme and to pri-miRNAs, and is required for the formation of a pre-microRNA (pre-miRNA), the initial step of microRNA (miRNA) biogenesis. The complex is composed of the double-stranded-RNA-specific RNase Drosha (also called RNASEN) and the RNA-binding protein DGCR8 (heme-free or heme-bound forms). Within the complex, DGCR8 function as a molecular anchor necessary for the recognition of pri-miRNA at dsRNA-ssRNA junction and directs RNASEN/Drosha to cleave the 3' and 5' strands of a stem-loop to release hairpin-shaped pre-miRNAs. Relationships: is a type of nuclear protein-containing complex [GO:0140513]; is a type of ribonuclease III complex [GO:1903095] References: PMID:16963499, PMID:17159994